{
  "gene_name": "TBC1 domain family member 12",
  "gene": "UniProtKB:O60347",
  "term_label": "autophagosome",
  "term_id": "GO:0005776",
  "gene_symbol": "TBC1D12"
}